{
  "gene": "UniProtKB:A6NFF2",
  "term_id": "UNKNOWN:0001",
  "gene_name": "Putative nucleosome assembly protein 1-like 6",
  "gene_symbol": "NAP1L6P",
  "term_label": "Unknown molecular function"
}